{
  "term_label": "protein export from nucleus",
  "gene_symbol": "CCHCR1",
  "gene_name": "Coiled-coil alpha-helical rod protein 1",
  "gene": "UniProtKB:Q8TD31",
  "term_id": "GO:0006611"
}